{
  "gene_symbol": "PRRX1",
  "gene_name": "Paired mesoderm homeobox protein 1",
  "term_id": "GO:0005634",
  "gene": "UniProtKB:P54821",
  "term_label": "nucleus"
}